{
  "term_id": "GO:0008821",
  "gene_name": "Crossover junction endonuclease MUS81",
  "gene": "UniProtKB:Q96NY9",
  "term_label": "crossover junction DNA endonuclease activity",
  "gene_symbol": "MUS81"
}